SCF-Hrt3/Pof7 ubiquitin ligase complex [GO:0097675] (cellular component) Definition: An SCF ubiquitin ligase complex in which the F-box protein is Hrt3 in S. cerevisiae (Pof7 in S. pombe). References: PMID:14747994, PMID:15147268 Sources: GOC:jd, GOC:vw Relationships: is a type of SCF ubiquitin ligase complex [GO:0019005]